3-deoxy-D-manno-octulosonate aldolase activity [GO:0047439] (molecular function) Definition: Catalysis of the reaction: 3-deoxy-D-manno-octulosonate = D-arabinose + pyruvate. Sources: EC:4.1.2.23, RHEA:23340 Also known as: 2-keto-3-deoxyoctonate aldolase activity, 2-keto-3-deoxyoctonic aldolase activity, 3-deoxy-D-manno-octulosonate D-arabinose-lyase (pyruvate-forming), 3-deoxy-D-manno-octulosonate D-arabinose-lyase activity, 3-deoxy-D-manno-octulosonic aldolase activity, 3-deoxyoctulosonic aldolase activity, KDOaldolase activity Relationships: is a type of aldehyde-lyase activity [GO:0016832]